{
  "gene_name": "Sorting nexin-15",
  "term_label": "plasma membrane",
  "term_id": "GO:0005886",
  "gene": "UniProtKB:Q9NRS6",
  "gene_symbol": "SNX15"
}